phosphoethanolamine N-methyltransferase activity [GO:0000234] (MF) Sources: EC:2.1.1.103 Also known as: S-adenosyl-L-methionine:ethanolamine-phosphate N-methyltransferase activity, phosphoethanolamine methyltransferase activity Relationships: is a type of N-methyltransferase activity [GO:0008170]; is a type of S-adenosylmethionine-dependent methyltransferase activity [GO:0008757] Definition: Catalysis of the reaction: S-adenosyl-L-methionine + ethanolamine phosphate = S-adenosyl-L-homocysteine + N-methylethanolamine phosphate.